{
  "gene": "UniProtKB:Q96M60",
  "gene_name": "Protein FAM227B",
  "gene_symbol": "FAM227B",
  "term_label": "Unknown cellular component",
  "term_id": "UNKNOWN:0003"
}